larval feeding behavior [GO:0030536] (biological process) Definition: Feeding behavior in a larval (immature) organism. Relationships: is a type of feeding behavior [GO:0007631]; is a type of larval behavior [GO:0030537] Sources: GOC:mah Note: See also the biological process term 'feeding behavior ; GO:0007631'. Also known as: larval feeding behaviour